{
  "gene_symbol": "FGGY",
  "gene_name": "FGGY carbohydrate kinase domain-containing protein",
  "gene": "UniProtKB:Q96C11",
  "term_label": "D-ribulokinase activity",
  "term_id": "GO:0019150"
}